{
  "term_id": "GO:0004705",
  "gene_symbol": "MAPK9",
  "gene_name": "Mitogen-activated protein kinase 9",
  "term_label": "JUN kinase activity",
  "gene": "UniProtKB:P45984"
}